{
  "term_label": "cytosol",
  "gene_symbol": "CRYZ",
  "gene_name": "Quinone oxidoreductase",
  "gene": "UniProtKB:Q08257",
  "term_id": "GO:0005829"
}